{
  "gene_name": "RNA-binding protein FXR1",
  "gene": "UniProtKB:P51114",
  "gene_symbol": "FXR1",
  "term_label": "cytoplasmic stress granule",
  "term_id": "GO:0010494"
}